{
  "gene_name": "Putative uncharacterized protein encoded by LINC02694",
  "gene_symbol": "LINC02694",
  "term_label": "Unknown biological process",
  "gene": "UniProtKB:Q8NAA6",
  "term_id": "UNKNOWN:0002"
}